{
  "gene_name": "Protocadherin beta-7",
  "term_label": "cell adhesion",
  "gene": "UniProtKB:Q9Y5E2",
  "gene_symbol": "PCDHB7",
  "term_id": "GO:0007155"
}